{
  "term_label": "junctional sarcoplasmic reticulum membrane",
  "gene_name": "Triadin",
  "gene": "UniProtKB:Q13061",
  "term_id": "GO:0014701",
  "gene_symbol": "TRDN"
}